piRNA binding [GO:0034584] (MF) Definition: Binding to a piRNA, a Piwi-associated RNA, a 24- to 30-nucleotide RNA derived from repeat or complex DNA sequence elements and processed by a Dicer-independent mechanism. Also known as: Piwi-associated RNA binding Relationships: is a type of GO:0061980 Sources: GOC:kmv